R3/R4 cell fate commitment [GO:0007464] (biological process) Definition: The process in which the R3/R4 photoreceptors commit to their cell fate. R3 and R4 are paired photoreceptors which contribute the outer rhabdomeres. References: PMID:3076112, PMID:3937883 Relationships: is a type of GO:0001752; BFO_0000050 establishment of ommatidial planar polarity [GO:0042067]; is part of R3/R4 cell differentiation [GO:0048056]